heptasaccharide transport [GO:2001104] (biological process) Definition: The directed movement of a heptasaccharideacetate into, out of or within a cell, or between cells, by means of some agent such as a transporter or pore. Regulation: regulated by regulation of heptasaccharide transport [GO:1900294]; negatively regulated by negative regulation of heptasaccharide transport [GO:1900295]; positively regulated by positive regulation of heptasaccharide transport [GO:1900296] Sources: GOC:mengo_curators Relationships: is a type of oligosaccharide transport [GO:0015772] Subtypes: GO:2001105